regulation of hepatic stellate cell migration [GO:0061869] (biological process) Relationships: is a type of regulation of fibroblast migration [GO:0010762]; regulates hepatic stellate cell migration [GO:0061868] Subtypes: positive regulation of hepatic stellate cell migration [GO:0061870], negative regulation of hepatic stellate cell migration [GO:0061871] References: PMID:24204762 Definition: Any process that modulates the frequency, rate or extent of hepatic stellate cell migration.